regulation of respiratory system process [GO:0044065] (biological process) Relationships: is a type of GO:0043576; is a type of regulation of system process [GO:0044057]; regulates respiratory system process [GO:0003016] Definition: Any process that modulates the frequency, rate or extent of a respiratory system process, an organ system process carried out by any of the organs or tissues of the respiratory system. Subtypes: regulation of respiratory gaseous exchange by nervous system process [GO:0002087] Sources: GOC:jl